{
  "gene_name": "S-formylglutathione hydrolase",
  "gene": "UniProtKB:P10768",
  "gene_symbol": "ESD",
  "term_id": "UNKNOWN:0002",
  "term_label": "Unknown biological process"
}